{
  "gene_name": "Potassium voltage-gated channel subfamily KQT member 1",
  "term_id": "GO:0015271",
  "gene": "UniProtKB:P51787",
  "term_label": "outward rectifier potassium channel activity",
  "gene_symbol": "KCNQ1"
}